{
  "gene_name": "Histone H2B type 1-J",
  "term_id": "GO:0061844",
  "term_label": "antimicrobial humoral immune response mediated by antimicrobial peptide",
  "gene_symbol": "H2BC11",
  "gene": "UniProtKB:P06899"
}